{
  "term_id": "GO:0003950",
  "gene_symbol": "PARP1",
  "term_label": "NAD+ poly-ADP-ribosyltransferase activity",
  "gene": "UniProtKB:P09874",
  "gene_name": "Poly [ADP-ribose] polymerase 1"
}